positive regulation of potassium ion import across plasma membrane [GO:1903288] (biological process) Also known as: positive regulation of potassium ion import, positive regulation of potassium import, positive regulation of potassium ion uptake, up regulation of potassium import, up regulation of potassium ion import, up regulation of potassium ion uptake, up-regulation of potassium import, up-regulation of potassium ion import, up-regulation of potassium ion uptake, upregulation of potassium import, upregulation of potassium ion import, upregulation of potassium ion uptake, activation of potassium import, activation of potassium ion import, activation of potassium ion uptake References: PMID:10636900 Sources: GOC:BHF, GOC:TermGenie, GOC:mtg_cardiac_conduct_nov11, GOC:rl, GO_REF:0000058 Definition: Any process that activates or increases the frequency, rate or extent of potassium ion import across the plasma membrane. Relationships: is a type of positive regulation of potassium ion transmembrane transport [GO:1901381]; is a type of regulation of potassium ion import [GO:1903286]; positively regulates potassium ion import across plasma membrane [GO:1990573]